{
  "gene": "UniProtKB:Q32M84",
  "term_id": "UNKNOWN:0003",
  "term_label": "Unknown cellular component",
  "gene_name": "BTB_POZ domain-containing protein 16",
  "gene_symbol": "BTBD16"
}